{
  "gene_name": "MICOS complex subunit MIC25",
  "gene": "UniProtKB:Q9BRQ6",
  "gene_symbol": "CHCHD6",
  "term_label": "cristae formation",
  "term_id": "GO:0042407"
}